{
  "gene_symbol": "SORT1",
  "term_id": "GO:0005794",
  "gene_name": "Sortilin",
  "gene": "UniProtKB:Q99523",
  "term_label": "Golgi apparatus"
}